{
  "term_label": "Unknown cellular component",
  "gene_symbol": "CLYBL",
  "gene_name": "Citramalyl-CoA lyase, mitochondrial",
  "term_id": "UNKNOWN:0003",
  "gene": "UniProtKB:Q8N0X4"
}